fourth ventricle development [GO:0021592] (BP) Sources: GOC:cls, GOC:dgh, GOC:dph, GOC:jid, GO_REF:0000021 Definition: The process whose specific outcome is the progression of the fourth ventricle over time, from its formation to the mature structure. The fourth ventricle is an irregularly shaped cavity in the rhombencephalon, between the medulla oblongata, the pons, and the isthmus in front, and the cerebellum behind. It is continuous with the central canal of the cord below and with the cerebral aqueduct above, and through its lateral and median apertures it communicates with the subarachnoid space. Relationships: is a type of anatomical structure development [GO:0048856]; is part of GO:0021591; is part of GO:0030902